{
  "gene_symbol": "CUEDC2",
  "term_id": "UNKNOWN:0002",
  "term_label": "Unknown biological process",
  "gene": "UniProtKB:Q9H467",
  "gene_name": "CUE domain-containing protein 2"
}